{
  "term_label": "Unknown molecular function",
  "gene_symbol": "TMEM130",
  "gene_name": "Transmembrane protein 130",
  "gene": "UniProtKB:Q8N3G9",
  "term_id": "UNKNOWN:0001"
}